positive regulation of proton-transporting ATP synthase activity, rotational mechanism [GO:1905273] (biological process) Relationships: is a type of positive regulation of ligase activity [GO:0051351]; is a type of positive regulation of cation channel activity [GO:2001259]; RO_0002213 proton-transporting ATP synthase activity, rotational mechanism [GO:0046933] References: PMID:21106936 Sources: GOC:TermGenie, GOC:als, GO_REF:0000059 Also known as: positive regulation of H+-transporting ATP synthase activity, positive regulation of hydrogen ion translocating F-type ATPase activity, positive regulation of hydrogen ion transporting ATP synthase activity, rotational mechanism, positive regulation of hydrogen ion transporting two-sector ATPase activity, up regulation of H+-transporting ATP synthase activity, up regulation of hydrogen ion translocating F-type ATPase activity, up regulation of hydrogen ion transporting ATP synthase activity, rotational mechanism, up regulation of hydrogen ion transporting two-sector ATPase activity, up regulation of proton-transporting ATP synthase activity, rotational mechanism, up-regulation of H+-transporting ATP synthase activity, up-regulation of hydrogen ion translocating F-type ATPase activity, up-regulation of hydrogen ion transporting ATP synthase activity, rotational mechanism, up-regulation of hydrogen ion transporting two-sector ATPase activity, up-regulation of proton-transporting ATP synthase activity, rotational mechanism, upregulation of H+-transporting ATP synthase activity, upregulation of hydrogen ion translocating F-type ATPase activity, upregulation of hydrogen ion transporting ATP synthase activity, rotational mechanism, upregulation of hydrogen ion transporting two-sector ATPase activity, upregulation of proton-transporting ATP synthase activity, rotational mechanism, activation of H+-transporting ATP synthase activity, activation of hydrogen ion translocating F-type ATPase activity, activation of hydrogen ion transporting ATP synthase activity, rotational mechanism, activation of hydrogen ion transporting two-sector ATPase activity, activation of proton-transporting ATP synthase activity, rotational mechanism Definition: Any process that activates or increases the frequency, rate or extent of proton-transporting ATP synthase activity, rotational mechanism.